{
  "term_label": "DNA-binding transcription factor activity, RNA polymerase II-specific",
  "term_id": "GO:0000981",
  "gene_symbol": "TFDP2",
  "gene": "UniProtKB:Q14188",
  "gene_name": "Transcription factor Dp-2"
}